(2R)-2-hydroxyacid dehydrogenase (NAD+) activity [GO:0140175] (molecular function) Definition: Catalysis of the reaction: a (2R)-2-hydroxycarboxylate + NAD+ = a 2-oxocarboxylate + NADH + H+. Subtypes: GO:0008720, (2R)-hydroxyphenylpyruvate reductase [NAD(P)H] activity [GO:0047995], phenyllactate dehydrogenase (NAD+) activity [GO:0097256] Relationships: is a type of oxidoreductase activity, acting on the CH-OH group of donors, NAD or NADP as acceptor [GO:0016616] Sources: RHEA:35643